{
  "term_label": "Unknown biological process",
  "gene": "UniProtKB:Q96MZ4",
  "gene_name": "Protein FAM218A",
  "term_id": "UNKNOWN:0002",
  "gene_symbol": "FAM218A"
}